{
  "gene_name": "Angiogenin",
  "term_id": "GO:0001525",
  "term_label": "angiogenesis",
  "gene": "UniProtKB:P03950",
  "gene_symbol": "ANG"
}